{
  "term_id": "GO:0007030",
  "gene_name": "Golgin subfamily A member 8B",
  "gene": "UniProtKB:A8MQT2",
  "term_label": "Golgi organization",
  "gene_symbol": "GOLGA8B"
}